secondary metabolite biosynthetic process [GO:0044550] (biological process) Also known as: secondary metabolite biosynthesis Regulation: regulated by regulation of secondary metabolite biosynthetic process [GO:1900376]; negatively regulated by GO:1900377; positively regulated by positive regulation of secondary metabolite biosynthetic process [GO:1900378] Relationships: is a type of GO:0009058; is_a GO:0019748 Subtypes: GO:0008055, toxin biosynthetic process [GO:0009403], phenylpropanoid biosynthetic process [GO:0009699], alkaloid biosynthetic process [GO:0009821], GO:0019290, GO:0019756, polyketide biosynthetic process [GO:0030639], asperthecin biosynthetic process [GO:0036184], penicillin biosynthetic process [GO:0042318], melanin biosynthetic process [GO:0042438], pheromone biosynthetic process [GO:0042811], orcinol biosynthetic process [GO:0046197], cichorine biosynthetic process [GO:0062032], GO:1900541, N',N'',N'''-triacetylfusarinine C biosynthetic process [GO:1900551], emericellamide biosynthetic process [GO:1900557], GO:1900563, diorcinol biosynthetic process [GO:1900572], emodin biosynthetic process [GO:1900575], gerfelin biosynthetic process [GO:1900578], (17Z)-protosta-17(20),24-dien-3beta-ol biosynthetic process [GO:1900581], o-orsellinic acid biosynthetic process [GO:1900584], arugosin biosynthetic process [GO:1900587], violaceol I biosynthetic process [GO:1900590], GO:1900593, (+)-kotanin biosynthetic process [GO:1900596], demethylkotanin biosynthetic process [GO:1900599], endocrocin biosynthetic process [GO:1900602], GO:1900605, tensidol B biosynthetic process [GO:1900608], emericellin biosynthetic process [GO:1900766], shamixanthone biosynthetic process [GO:1900793], GO:1900799, cspyrone B1 biosynthetic process [GO:1900802], helvolic acid biosynthetic process [GO:1900812], monodictyphenone biosynthetic process [GO:1900815], ochratoxin A biosynthetic process [GO:1900818], orlandin biosynthetic process [GO:1900821] Definition: The chemical reactions and pathways resulting in the formation of secondary metabolites, the compounds that are not necessarily required for growth and maintenance of cells, and are often unique to a taxon. Sources: GOC:jl